{
  "gene_symbol": "OTUB2",
  "gene": "UniProtKB:Q96DC9",
  "term_id": "GO:0043130",
  "gene_name": "Ubiquitin thioesterase OTUB2",
  "term_label": "ubiquitin binding"
}